{
  "gene": "UniProtKB:Q8TF46",
  "gene_name": "DIS3-like exonuclease 1",
  "term_label": "mRNA catabolic process",
  "gene_symbol": "DIS3L",
  "term_id": "GO:0006402"
}